{
  "term_label": "serine-type endopeptidase inhibitor activity",
  "gene_name": "Serpin E3",
  "term_id": "GO:0004867",
  "gene": "UniProtKB:A8MV23",
  "gene_symbol": "SERPINE3"
}